choline catabolic process [GO:0042426] (biological process) Relationships: is a type of GO:0019695; is a type of biogenic amine catabolic process [GO:0042402] Definition: The chemical reactions and pathways resulting in the breakdown of choline (2-hydroxyethyltrimethylammonium), an amino alcohol that occurs widely in living organisms as a constituent of certain types of phospholipids and in the neurotransmitter acetylcholine. Sources: GOC:jl, ISBN:0192801023 Also known as: choline breakdown, choline catabolism, choline degradation